{
  "term_label": "negative regulation of mitochondrial outer membrane permeabilization involved in apoptotic signaling pathway",
  "gene": "UniProtKB:Q2QL34",
  "gene_name": "Mpv17-like protein",
  "gene_symbol": "MPV17L",
  "term_id": "GO:1901029"
}